{
  "term_label": "glycerol channel activity",
  "gene_symbol": "AQP9",
  "term_id": "GO:0015254",
  "gene": "UniProtKB:O43315",
  "gene_name": "Aquaporin-9"
}